{
  "gene_name": "NAD-dependent protein deacylase sirtuin-5, mitochondrial",
  "term_label": "protein-malonyllysine demalonylase activity",
  "gene": "UniProtKB:Q9NXA8",
  "gene_symbol": "SIRT5",
  "term_id": "GO:0036054"
}